{
  "gene_name": "Ryanodine receptor 2",
  "term_label": "sarcoplasmic reticulum membrane",
  "gene_symbol": "RYR2",
  "term_id": "GO:0033017",
  "gene": "UniProtKB:Q92736"
}